atrial cardiac muscle cell membrane repolarization [GO:0099624] (biological process) Definition: The process in which ions are transported across the plasma membrane of an atrial cardiac muscle cell such that the membrane potential changes in the repolarizing direction, toward the steady state potential. For example, the repolarization during an action potential is from a positive membrane potential towards a negative resting potential. Sources: GOC:BHF Relationships: is a type of cardiac muscle cell membrane repolarization [GO:0099622] Subtypes: membrane repolarization during atrial cardiac muscle cell action potential [GO:0098914] Regulation: regulated by regulation of atrial cardiac muscle cell membrane repolarization [GO:0060372]